{
  "gene_symbol": "KIAA1755",
  "gene_name": "Uncharacterized protein KIAA1755",
  "gene": "UniProtKB:Q5JYT7",
  "term_label": "extrinsic component of membrane",
  "term_id": "GO:0019898"
}